{
  "gene_symbol": "OLR1",
  "gene": "UniProtKB:P78380",
  "gene_name": "Oxidized low-density lipoprotein receptor 1",
  "term_id": "GO:0005041",
  "term_label": "low-density lipoprotein particle receptor activity"
}